{
  "term_label": "lysosomal lumen acidification",
  "gene_name": "Battenin",
  "gene_symbol": "CLN3",
  "term_id": "GO:0007042",
  "gene": "UniProtKB:Q13286"
}